{
  "term_id": "GO:0050830",
  "gene_symbol": "RNASE9",
  "gene": "UniProtKB:P60153",
  "term_label": "defense response to Gram-positive bacterium",
  "gene_name": "Inactive ribonuclease-like protein 9"
}